{
  "term_label": "replication fork processing",
  "gene_symbol": "MMS22L",
  "gene": "UniProtKB:Q6ZRQ5",
  "gene_name": "Protein MMS22-like",
  "term_id": "GO:0031297"
}